{
  "term_id": "UNKNOWN:0001",
  "gene_name": "Pregnancy-specific beta-1-glycoprotein 9",
  "gene_symbol": "PSG9",
  "term_label": "Unknown molecular function",
  "gene": "UniProtKB:Q00887"
}